{
  "term_label": "lysosomal membrane",
  "term_id": "GO:0005765",
  "gene_symbol": "RNF152",
  "gene": "UniProtKB:Q8N8N0",
  "gene_name": "E3 ubiquitin-protein ligase RNF152"
}